{
  "term_id": "GO:0006357",
  "term_label": "regulation of transcription by RNA polymerase II",
  "gene_symbol": "ZNF778",
  "gene": "UniProtKB:Q96MU6",
  "gene_name": "Zinc finger protein 778"
}